{
  "gene_name": "Putative tripartite motif-containing protein 51G",
  "gene_symbol": "TRIM51G",
  "gene": "UniProtKB:A0A3B3IT33",
  "term_label": "ubiquitin protein ligase activity",
  "term_id": "GO:0061630"
}